{
  "gene_symbol": "LYG1",
  "gene_name": "Lysozyme g-like protein 1",
  "term_id": "GO:0050830",
  "term_label": "defense response to Gram-positive bacterium",
  "gene": "UniProtKB:Q8N1E2"
}